{
  "term_id": "GO:0019985",
  "gene_symbol": "PCLAF",
  "term_label": "translesion synthesis",
  "gene": "UniProtKB:Q15004",
  "gene_name": "PCNA-associated factor"
}